{
  "gene": "UniProtKB:Q96Q42",
  "term_id": "GO:0005813",
  "gene_symbol": "ALS2",
  "gene_name": "Alsin",
  "term_label": "centrosome"
}